cholesterol biosynthetic process via desmosterol [GO:0033489] (biological process) Also known as: cholesterol anabolism via desmosterol, cholesterol biosynthesis via desmosterol, cholesterol formation via desmosterol, cholesterol synthesis via desmosterol Relationships: is a type of cholesterol biosynthetic process [GO:0006695] Definition: The chemical reactions and pathways resulting in the formation of cholesterol, cholest-5-en-3 beta-ol, via the intermediate desmosterol. Sources: GOC:mah, MetaCyc:PWY66-4